{
  "gene_name": "Small ribosomal subunit protein uS9m",
  "term_label": "RNA binding",
  "gene_symbol": "MRPS9",
  "gene": "UniProtKB:P82933",
  "term_id": "GO:0003723"
}